regulation of memory T cell differentiation [GO:0043380] (biological process) Definition: Any process that modulates the frequency, rate, or extent of memory T cell differentiation. Sources: ISBN:0781735149 Also known as: regulation of memory T lymphocyte differentiation, regulation of memory T-cell differentiation, regulation of memory T-lymphocyte differentiation, regulation of memory T cell development Note: Note that immunologists typically use the word 'development' to refer to cells of B or T cell lineages undergoing the process that GO describes as 'cell differentiation'. Relationships: is a type of regulation of immune effector process [GO:0002697]; is a type of GO:0045580; is a type of GO:0050776; regulates memory T cell differentiation [GO:0043379] Subtypes: negative regulation of memory T cell differentiation [GO:0043381], positive regulation of memory T cell differentiation [GO:0043382]